negative regulation of tensidol B biosynthetic process [GO:1900711] (biological process) Sources: GOC:TermGenie, GOC:di Relationships: is a type of negative regulation of amide metabolic process [GO:0034249]; is a type of negative regulation of small molecule metabolic process [GO:0062014]; is a type of GO:1900377; is a type of GO:1900710; RO_0002212 tensidol B biosynthetic process [GO:1900608] Also known as: down regulation of tensidol B anabolism, down regulation of tensidol B biosynthesis, down regulation of tensidol B biosynthetic process, down regulation of tensidol B formation, down regulation of tensidol B synthesis, down-regulation of tensidol B anabolism, down-regulation of tensidol B biosynthesis, down-regulation of tensidol B biosynthetic process, down-regulation of tensidol B formation, down-regulation of tensidol B synthesis, downregulation of tensidol B anabolism, downregulation of tensidol B biosynthesis, downregulation of tensidol B biosynthetic process, downregulation of tensidol B formation, downregulation of tensidol B synthesis, inhibition of tensidol B anabolism, inhibition of tensidol B biosynthesis, inhibition of tensidol B formation, inhibition of tensidol B synthesis, negative regulation of tensidol B anabolism, negative regulation of tensidol B biosynthesis, negative regulation of tensidol B formation, negative regulation of tensidol B synthesis, inhibition of tensidol B biosynthetic process Definition: Any process that stops, prevents or reduces the frequency, rate or extent of tensidol B biosynthetic process.